{
  "gene_symbol": "GCFC2",
  "term_id": "GO:0005634",
  "gene_name": "Intron Large complex component GCFC2",
  "term_label": "nucleus",
  "gene": "UniProtKB:P16383"
}